{
  "gene_symbol": "TAP1",
  "term_id": "GO:0015433",
  "gene": "UniProtKB:Q03518",
  "term_label": "ABC-type peptide antigen transporter activity",
  "gene_name": "Antigen peptide transporter 1"
}